{
  "term_id": "GO:0005744",
  "gene_symbol": "TIMM17A",
  "term_label": "TIM23 mitochondrial import inner membrane translocase complex",
  "gene": "UniProtKB:Q99595",
  "gene_name": "Mitochondrial import inner membrane translocase subunit Tim17-A"
}